{
  "gene_symbol": "PALLD",
  "term_id": "GO:0030424",
  "gene": "UniProtKB:Q8WX93",
  "gene_name": "Palladin",
  "term_label": "axon"
}